{
  "gene": "UniProtKB:P04440",
  "term_id": "GO:0031902",
  "gene_symbol": "HLA-DPB1",
  "gene_name": "HLA class II histocompatibility antigen, DP beta 1 chain",
  "term_label": "late endosome membrane"
}